{
  "term_label": "cell adhesion molecule binding",
  "gene_name": "Protocadherin alpha-11",
  "gene": "UniProtKB:Q9Y5I1",
  "term_id": "GO:0050839",
  "gene_symbol": "PCDHA11"
}